{
  "gene": "UniProtKB:Q9HCR9",
  "gene_symbol": "PDE11A",
  "term_label": "Unknown cellular component",
  "term_id": "UNKNOWN:0003",
  "gene_name": "Dual 3',5'-cyclic-AMP and -GMP phosphodiesterase 11A"
}